{
  "gene": "UniProtKB:A6NHN0",
  "term_label": "extracellular matrix organization",
  "gene_name": "Otolin-1",
  "term_id": "GO:0030198",
  "gene_symbol": "OTOL1"
}